{
  "term_label": "Unknown cellular component",
  "gene": "UniProtKB:A0A1B0GTG8",
  "term_id": "UNKNOWN:0003",
  "gene_symbol": "LOC105372440",
  "gene_name": "Uncharacterized protein"
}